{
  "term_id": "UNKNOWN:0003",
  "term_label": "Unknown cellular component",
  "gene_name": "Zinc finger protein 202",
  "gene": "UniProtKB:O95125",
  "gene_symbol": "ZNF202"
}